{
  "gene_symbol": "BIRC6",
  "gene": "UniProtKB:Q9NR09",
  "term_label": "negative regulation of apoptotic process",
  "term_id": "GO:0043066",
  "gene_name": "Baculoviral IAP repeat-containing protein 6"
}